{
  "gene": "UniProtKB:Q12798",
  "term_id": "GO:0005634",
  "gene_symbol": "CETN1",
  "gene_name": "Centrin-1",
  "term_label": "nucleus"
}